symporter activity [GO:0015293] (molecular function) Subtypes: GO:0015294 Also known as: cotransporter activity, porter activity, symport Relationships: is a type of secondary active transmembrane transporter activity [GO:0015291] References: PMID:10839820 Sources: GOC:mtg_transport, ISBN:0815340729 Definition: Enables the active transport of a solute across a membrane by a mechanism whereby two or more species are transported together in the same direction in a tightly coupled process not directly linked to a form of energy other than chemiosmotic energy.